{
  "term_id": "GO:0006906",
  "gene_name": "Syntaxin-16",
  "gene_symbol": "STX16",
  "gene": "UniProtKB:O14662",
  "term_label": "vesicle fusion"
}